{
  "term_id": "GO:0005737",
  "term_label": "cytoplasm",
  "gene_name": "Tubulin alpha chain-like 3",
  "gene_symbol": "TUBAL3",
  "gene": "UniProtKB:A6NHL2"
}